N-acetylneuraminate metabolic process [GO:0006054] (biological process) Also known as: sialic acid metabolic process, sialic acid metabolism, N-acetylneuraminate metabolism Relationships: is a type of amino sugar metabolic process [GO:0006040]; is a type of carboxylic acid metabolic process [GO:0019752]; is a type of amide metabolic process [GO:0043603] Subtypes: N-acetylneuraminate catabolic process [GO:0019262], GO:0046380 Sources: ISBN:0198506732 Definition: The chemical reactions and pathways involving N-acetylneuraminate, the anion of 5-(acetylamino)-3,5-dideoxy-D-glycero-D-galacto-non-3-ulosonic acid.